L-serine-phosphatidylcholine phosphatidyltransferase activity [GO:0106258] (molecular function) Relationships: is a type of phosphotransferase activity, for other substituted phosphate groups [GO:0016780] References: PMID:19014349 Sources: RHEA:45088 Definition: Catalysis of the reaction: a 1,2-diacyl-sn-glycero-3-phosphocholine + L-serine = 1,2-diacyl-sn-glycero-3-phospho-L-serine + choline.